{
  "gene_symbol": "AOAH",
  "term_label": "acyloxyacyl hydrolase activity",
  "gene_name": "Acyloxyacyl hydrolase",
  "term_id": "GO:0050528",
  "gene": "UniProtKB:P28039"
}